regulation of telomerase catalytic core complex assembly [GO:1904882] (BP) Definition: Any process that modulates the frequency, rate or extent of telomerase catalytic core complex assembly. References: PMID:26586433 Sources: GOC:BHF, GOC:BHF_telomere, GOC:TermGenie, GOC:rph, GO_REF:0000058 Subtypes: GO:1904883, positive regulation of telomerase catalytic core complex assembly [GO:1904884] Relationships: is a type of GO:0043254; regulates telomerase catalytic core complex assembly [GO:1904868] Also known as: regulation of telomerase catalytic core complex formation, regulation of TERT-TERC complex assembly, regulation of TERT-TERC complex formation